{
  "gene": "UniProtKB:O75683",
  "gene_symbol": "SURF6",
  "term_label": "ribosomal large subunit biogenesis",
  "term_id": "GO:0042273",
  "gene_name": "Surfeit locus protein 6"
}